positive regulation of hepatocyte growth factor production [GO:0032726] (biological process) Definition: Any process that activates or increases the frequency, rate, or extent of hepatocyte growth factor production. Also known as: positive regulation of HGF production, positive regulation of scatter factor production, up regulation of hepatocyte growth factor production, up-regulation of hepatocyte growth factor production, upregulation of hepatocyte growth factor production, activation of hepatocyte growth factor production, positive regulation of hepatocyte growth factor biosynthetic process, stimulation of hepatocyte growth factor production Relationships: is a type of positive regulation of cytokine production [GO:0001819]; is a type of regulation of hepatocyte growth factor production [GO:0032646]; is a type of positive regulation of protein metabolic process [GO:0051247]; positively regulates hepatocyte growth factor production [GO:0032605] References: PMID:1838014 Sources: GOC:mah